{
  "gene": "UniProtKB:Q96QE3",
  "gene_symbol": "ATAD5",
  "gene_name": "ATPase family AAA domain-containing protein 5",
  "term_id": "UNKNOWN:0002",
  "term_label": "Unknown biological process"
}